symbiont-mediated suppression of host antigen processing and presentation [GO:0039588] (biological process) Also known as: suppression by virus of host antigen processing and presentation Sources: VZ:815 Definition: A process by which a symbiont inhibits or disrupts the normal processing and presentation of a peptide antigen on its cell surface in association with an MHC protein complex. Relationships: is a type of symbiont-mediated suppression of host adaptive immune response [GO:0039504] Subtypes: symbiont-mediated suppression of host antigen processing and presentation of peptide antigen via MHC class II [GO:0039505], symbiont-mediated suppression of host antigen processing and presentation of peptide antigen via MHC class I [GO:0046776]